{
  "term_label": "heme binding",
  "gene": "UniProtKB:Q9NRV9",
  "gene_symbol": "HEBP1",
  "term_id": "GO:0020037",
  "gene_name": "Heme-binding protein 1"
}